translational initiation [GO:0006413] (BP) Sources: ISBN:019879276X Definition: The process preceding formation of the peptide bond between the first two amino acids of a protein. This includes the formation of a complex of the ribosome, mRNA or circRNA, and an initiation complex that contains the first aminoacyl-tRNA. Also known as: biopolymerisation, biopolymerization, protein synthesis initiation, translation initiation Subtypes: cytoplasmic translational initiation [GO:0002183], mitochondrial translational initiation [GO:0070124] Relationships: is a type of metabolic process [GO:0008152]; is part of translation [GO:0006412]; BFO_0000051 formation of translation initiation ternary complex [GO:0001677] Regulation: regulated by regulation of translational initiation [GO:0006446]; negatively regulated by GO:0045947; positively regulated by positive regulation of translational initiation [GO:0045948]